{
  "gene_symbol": "BTBD17",
  "term_id": "UNKNOWN:0002",
  "gene": "UniProtKB:A6NE02",
  "term_label": "Unknown biological process",
  "gene_name": "BTB_POZ domain-containing protein 17"
}